{
  "term_id": "GO:0005737",
  "term_label": "cytoplasm",
  "gene_name": "Bifunctional glutamate_proline--tRNA ligase",
  "gene_symbol": "EPRS1",
  "gene": "UniProtKB:P07814"
}